{
  "term_label": "modulation of chemical synaptic transmission",
  "gene_symbol": "BTBD9",
  "gene": "UniProtKB:Q96Q07",
  "term_id": "GO:0050804",
  "gene_name": "BTB_POZ domain-containing protein 9"
}